thymidine phosphorylase activity [GO:0009032] (molecular function) Definition: Catalysis of the reaction: thymidine + phosphate = thymine + 2-deoxy-D-ribose 1-phosphate. Sources: RHEA:16037 Also known as: pyrimidine phosphorylase activity, thymidine-orthophosphate deoxyribosyltransferase activity, thymidine:phosphate deoxy-D-ribosyltransferase activity, thymidine:phosphate deoxy-alpha-D-ribosyltransferase activity Relationships: is a type of pyrimidine-nucleoside phosphorylase activity [GO:0016154]